negative regulation of phosphorus utilization [GO:0045942] (biological process) Relationships: is a type of regulation of phosphorus utilization [GO:0006795]; is a type of negative regulation of phosphorus metabolic process [GO:0010563]; negatively regulates phosphorus utilization [GO:0006794] Also known as: down regulation of phosphorus utilization, down-regulation of phosphorus utilization, downregulation of phosphorus utilization, inhibition of phosphorus utilization Sources: GOC:go_curators Definition: Any process that stops, prevents, or reduces the frequency, rate or extent of phosphorus utilization.